{
  "gene_name": "[Pyruvate dehydrogenase (acetyl-transferring)] kinase isozyme 4, mitochondrial",
  "gene_symbol": "PDK4",
  "gene": "UniProtKB:Q16654",
  "term_label": "pyruvate dehydrogenase (acetyl-transferring) kinase activity",
  "term_id": "GO:0004740"
}